{
  "gene": "UniProtKB:Q9BWG4",
  "gene_symbol": "SSBP4",
  "term_id": "GO:0045944",
  "gene_name": "Single-stranded DNA-binding protein 4",
  "term_label": "positive regulation of transcription by RNA polymerase II"
}